negative regulation of Golgi to plasma membrane protein transport [GO:0042997] (biological process) Also known as: down regulation of Golgi to plasma membrane protein transport, down-regulation of Golgi to plasma membrane protein transport, downregulation of Golgi to plasma membrane protein transport, inhibition of Golgi to plasma membrane protein transport Definition: Any process that stops, prevents, or reduces the frequency, rate or extent of the transport of proteins from the Golgi to the plasma membrane. Relationships: is a type of regulation of Golgi to plasma membrane protein transport [GO:0042996]; is a type of negative regulation of protein transport [GO:0051224]; is a type of negative regulation of protein localization to plasma membrane [GO:1903077]; negatively regulates Golgi to plasma membrane protein transport [GO:0043001] Sources: GOC:jl